{
  "gene_symbol": "CHCHD2",
  "gene_name": "Coiled-coil-helix-coiled-coil-helix domain-containing protein 2",
  "term_label": "positive regulation of transcription by RNA polymerase II",
  "gene": "UniProtKB:Q9Y6H1",
  "term_id": "GO:0045944"
}